{
  "gene_symbol": "IL19",
  "gene": "UniProtKB:Q9UHD0",
  "gene_name": "Interleukin-19",
  "term_label": "immune response",
  "term_id": "GO:0006955"
}